{
  "gene": "UniProtKB:Q8IYX3",
  "term_label": "Unknown biological process",
  "gene_symbol": "CCDC116",
  "term_id": "UNKNOWN:0002",
  "gene_name": "Coiled-coil domain-containing protein 116"
}